{
  "gene_name": "Diphthine methyltransferase",
  "term_id": "GO:0017183",
  "term_label": "protein histidyl modification to diphthamide",
  "gene_symbol": "DPH7",
  "gene": "UniProtKB:Q9BTV6"
}